{
  "gene_symbol": "PLAC8",
  "gene_name": "Placenta-specific gene 8 protein",
  "gene": "UniProtKB:Q9NZF1",
  "term_id": "UNKNOWN:0003",
  "term_label": "Unknown cellular component"
}